negative regulation of norepinephrine secretion [GO:0010700] (biological process) Relationships: is a type of regulation of norepinephrine secretion [GO:0014061]; is a type of negative regulation of catecholamine secretion [GO:0033604]; negatively regulates norepinephrine secretion [GO:0048243] Sources: GOC:dph, GOC:tb Definition: Any process that decreases the frequency, rate or extent of the regulated release of norepinephrine.